chemical homeostasis [GO:0048878] (biological process) Sources: GOC:isa_complete Definition: Any biological process involved in the maintenance of an internal steady state of a chemical. Subtypes: carbohydrate homeostasis [GO:0033500], monoatomic ion homeostasis [GO:0050801], intracellular chemical homeostasis [GO:0055082], lipid homeostasis [GO:0055088], inorganic ion homeostasis [GO:0098771], ascorbate homeostasis [GO:0140576], multicellular organismal-level chemical homeostasis [GO:0140962] Relationships: is a type of GO:0042592